{
  "gene_name": "Ubiquitin carboxyl-terminal hydrolase 8",
  "term_id": "GO:0030496",
  "gene": "UniProtKB:P40818",
  "gene_symbol": "USP8",
  "term_label": "midbody"
}